{
  "gene_name": "Large ribosomal subunit protein mL41",
  "term_id": "GO:0005762",
  "gene_symbol": "MRPL41",
  "gene": "UniProtKB:Q8IXM3",
  "term_label": "mitochondrial large ribosomal subunit"
}